{
  "gene": "UniProtKB:Q9P0U4",
  "term_id": "GO:0045893",
  "term_label": "positive regulation of DNA-templated transcription",
  "gene_name": "CXXC-type zinc finger protein 1",
  "gene_symbol": "CXXC1"
}